{
  "term_id": "GO:0005634",
  "gene_symbol": "DCLK3",
  "term_label": "nucleus",
  "gene_name": "Serine_threonine-protein kinase DCLK3",
  "gene": "UniProtKB:Q9C098"
}